{
  "term_label": "nitric oxide mediated signal transduction",
  "gene_name": "Nitric oxide synthase, inducible",
  "gene_symbol": "NOS2",
  "gene": "UniProtKB:P35228",
  "term_id": "GO:0007263"
}